{
  "gene": "UniProtKB:P10082",
  "gene_symbol": "PYY",
  "term_label": "neuropeptide signaling pathway",
  "gene_name": "Peptide YY",
  "term_id": "GO:0007218"
}